male analia development [GO:0045496] (biological process) References: PMID:11494318 Sources: GOC:mtg_sensu Definition: The process whose specific outcome is the progression of the analia of the male over time, from formation to the mature structure. The analia is the posterior-most vertral appendage that develops from the genital disc. An example of this process is found in Drosophila melanogaster. Relationships: is a type of GO:0007487